protein localization to spore cell wall [GO:0099614] (biological process) Also known as: protein targeting to spore cell wall Sources: GOC:dos Definition: A process in which a protein is transported, tethered to or otherwise maintained in a spore cell wall. Subtypes: GO:1904853 Relationships: is a type of GO:1990778